{
  "gene": "UniProtKB:Q5VST6",
  "term_label": "palmitoyl-(protein) hydrolase activity",
  "gene_symbol": "ABHD17B",
  "gene_name": "Alpha_beta hydrolase domain-containing protein 17B",
  "term_id": "GO:0008474"
}